{
  "term_label": "Unknown molecular function",
  "term_id": "UNKNOWN:0001",
  "gene": "UniProtKB:Q9Y4H4",
  "gene_symbol": "GPSM3",
  "gene_name": "G-protein-signaling modulator 3"
}